{
  "gene": "UniProtKB:Q9UDX3",
  "gene_name": "SEC14-like protein 4",
  "term_label": "Unknown biological process",
  "term_id": "UNKNOWN:0002",
  "gene_symbol": "SEC14L4"
}